endocytic hemoglobin import into cell [GO:0020028] (biological process) Relationships: is a type of GO:0006898; is a type of GO:0015031; is a type of protein localization to organelle [GO:0033365]; is_a GO:0072594 Sources: GOC:mb Also known as: haemoglobin uptake, hemoglobin uptake, endocytic hemoglobin import Definition: The directed movement of hemoglobin into a cell by receptor-mediated endocytosis.